{
  "term_id": "GO:0008320",
  "gene_name": "Protein transport protein Sec61 subunit alpha isoform 2",
  "gene_symbol": "SEC61A2",
  "term_label": "protein transmembrane transporter activity",
  "gene": "UniProtKB:Q9H9S3"
}